inositol-1,3,4,5,6-pentakisphosphate 2-kinase activity [GO:0035299] (molecular function) Relationships: is a type of GO:0120517 Definition: Catalysis of the reaction: 1D-myo-inositol 1,3,4,5,6-pentakisphosphate + ATP = 1D-myo-inositol hexakisphosphate + ADP + H+. Also known as: inositol pentakisphosphate 2-kinase activity, IP5 2-kinase activity, Ins(1,3,4,5,6)P5 2-kinase activity, inositol hexakisphosphate synthase, inositol polyphosphate kinase activity, inositol-pentakisphosphate 2-kinase activity Sources: RHEA:20313